{
  "gene_symbol": "TXNDC15",
  "term_id": "GO:0005929",
  "gene": "UniProtKB:Q96J42",
  "gene_name": "Thioredoxin domain-containing protein 15",
  "term_label": "cilium"
}